neuregulin receptor activity [GO:0038131] (molecular function) Relationships: is a type of transmembrane signaling receptor activity [GO:0004888]; has part neuregulin binding [GO:0038132] Note: Consider also annotating to 'ERBB3 signaling pathway ; GO:0038129' and/or 'ERBB4 signaling pathway ; GO:0038130'. Also known as: NRG receptor activity, NRG1 receptor activity, NRG2 receptor activity Definition: Combining with a neuregulin, a member of the EGF family of growth factors, and transmitting the signal from one side of the membrane to the other to initiate a change in cell activity. References: PMID:16460914, PMID:20672328 Sources: GOC:bf, GOC:signaling